{
  "gene_symbol": "TBC1D2",
  "term_id": "GO:0005886",
  "term_label": "plasma membrane",
  "gene_name": "TBC1 domain family member 2A",
  "gene": "UniProtKB:Q9BYX2"
}